{
  "term_label": "positive regulation of cell migration",
  "gene": "UniProtKB:Q6UQ28",
  "gene_name": "Placenta-expressed transcript 1 protein",
  "gene_symbol": "PLET1",
  "term_id": "GO:0030335"
}